regulation of nucleoside transport [GO:0032242] (biological process) Definition: Any process that modulates the frequency, rate or extent of the directed movement of a nucleoside into, out of or within a cell, or between cells, by means of some agent such as a transporter or pore. Subtypes: negative regulation of nucleoside transport [GO:0032243], positive regulation of nucleoside transport [GO:0032244], GO:0032245, regulation of pyrimidine nucleoside transport [GO:0032246] Relationships: is a type of regulation of nucleobase-containing compound transport [GO:0032239]; regulates GO:0015858 Sources: GOC:mah